methylthiol:coenzyme M methyltransferase complex [GO:0044680] (cellular component) Also known as: methylthiol coenzyme M methyl transferase complex, methylthiol:CoM methyltransferase complex, methylthiol:coenzyme M methyl transferase complex Definition: A protein complex of two polypeptides which catalyzes the transfer of methyl group from methylthiol to coenzyme M during methanogenesis. References: PMID:11073950, PMID:9371433 Sources: GOC:mengo_curators Relationships: is a type of GO:0034708